ureter smooth muscle cell differentiation [GO:0072193] (biological process) Regulation: regulated by regulation of ureter smooth muscle cell differentiation [GO:2000061]; RO_0002212 by negative regulation of ureter smooth muscle cell differentiation [GO:2000062]; positively regulated by positive regulation of ureter smooth muscle cell differentiation [GO:2000063] Definition: The process in which a relatively unspecialized cell acquires specialized features of a smooth muscle cell in the ureter. Sources: GOC:mtg_kidney_jan10 Relationships: is a type of smooth muscle cell differentiation [GO:0051145]; is part of ureter smooth muscle development [GO:0072191]